{
  "gene_name": "CATR tumorigenic conversion 1 protein",
  "gene": "UniProtKB:Q13166",
  "term_id": "UNKNOWN:0002",
  "gene_symbol": "CATR1",
  "term_label": "Unknown biological process"
}